{
  "gene": "UniProtKB:Q9BTU6",
  "term_label": "plasma membrane",
  "gene_symbol": "PI4K2A",
  "gene_name": "Phosphatidylinositol 4-kinase type 2-alpha",
  "term_id": "GO:0005886"
}